{
  "gene": "UniProtKB:P01215",
  "gene_name": "Glycoprotein hormones alpha chain",
  "term_label": "extracellular space",
  "term_id": "GO:0005615",
  "gene_symbol": "CGA"
}